{
  "gene_symbol": "TRIM16",
  "term_id": "UNKNOWN:0003",
  "gene": "UniProtKB:O95361",
  "gene_name": "Tripartite motif-containing protein 16",
  "term_label": "Unknown cellular component"
}